polyuridylation-dependent mRNA catabolic process [GO:1990074] (biological process) References: PMID:23503588 Sources: GOC:vw Definition: The chemical reactions and pathways resulting in the breakdown of a messenger RNA (mRNA) molecule, initiated by the enzymatic addition of a sequence of uridylyl residues (polyuridylation) at the 3' end of the target mRNA. Relationships: is a type of mRNA catabolic process [GO:0006402]; is a type of GO:0043632; is a type of mRNA destabilization [GO:0061157]